cell growth [GO:0016049] (biological process) Subtypes: pseudohyphal growth [GO:0007124], multidimensional cell growth [GO:0009825], unidimensional cell growth [GO:0009826], developmental cell growth [GO:0048588], isotropic cell growth [GO:0051210], anisotropic cell growth [GO:0051211] Also known as: cellular growth, growth of cell, cell expansion, metabolic process resulting in cell growth, metabolism resulting in cell growth, non-developmental cell growth, non-developmental growth of a unicellular organism Definition: The process in which a cell irreversibly increases in size over time by accretion and biosynthetic production of matter similar to that already present. Sources: GOC:ai Regulation: regulated by regulation of cell growth [GO:0001558]; positively regulated by positive regulation of cell growth [GO:0030307]; negatively regulated by GO:0030308 Relationships: is a type of cellular process [GO:0009987]; is a type of GO:0040007